{
  "gene_symbol": "ADAMTSL4-AS1",
  "term_label": "Unknown cellular component",
  "gene_name": "Uncharacterized protein ADAMTSL4-AS1",
  "term_id": "UNKNOWN:0003",
  "gene": "UniProtKB:Q5T5F5"
}